negative regulation of SREBP signaling pathway in response to increased oxygen levels [GO:0038175] (biological process) References: PMID:22017871 Sources: GOC:al Relationships: is a type of negative regulation of SREBP signaling pathway [GO:2000639]; is part of cellular response to increased oxygen levels [GO:0036295] Also known as: negative regulation of SREBP-mediated signaling pathway in response to increased oxygen levels, negative regulation of SREBP-mediated signaling pathway in presence of oxygen Definition: Any process that stops, prevents or reduces the frequency, rate or extent of the SREBP signaling pathway in response to an increase in oxygen levels.